{
  "term_id": "GO:0042995",
  "gene_symbol": "ACTN1",
  "gene": "UniProtKB:P12814",
  "gene_name": "Alpha-actinin-1",
  "term_label": "cell projection"
}